intracellular chloride ion homeostasis [GO:0030644] (biological process) Also known as: cellular chloride ion homeostasis Relationships: is a type of GO:0030002; is a type of GO:0055064 Sources: GOC:mah Definition: A homeostatic process involved in the maintenance of a steady state level of chloride ions within a cell.